{
  "gene_name": "Putative transmembrane protein INAFM2",
  "gene_symbol": "INAFM2",
  "term_id": "UNKNOWN:0001",
  "gene": "UniProtKB:P0DMQ5",
  "term_label": "Unknown molecular function"
}